cysteine desulfurase activity [GO:0031071] (molecular function) Also known as: IscS, L-cysteine:enzyme cysteine sulfurtransferase activity, NIFS, SufS, cysteine desulfurylase activity Relationships: is a type of GO:0016783 Definition: Catalysis of the reaction: L-cysteine + [enzyme]-cysteine = L-alanine + [enzyme]-S-sulfanylcysteine. Sources: EC:2.8.1.7